type I hypersensitivity [GO:0016068] (biological process) Regulation: regulated by regulation of type I hypersensitivity [GO:0001810]; negatively regulated by negative regulation of type I hypersensitivity [GO:0001811]; positively regulated by GO:0001812 Note: Note that localized and systemic anaphylaxis is usually a result of type I hypersensitivity. Sources: GOC:add, ISBN:0781735149 Subtypes: type I hypersensitivity mediated by mast cells [GO:0002558], GO:0002559 Relationships: is a type of hypersensitivity [GO:0002524]; is a type of immunoglobulin mediated immune response [GO:0016064] Also known as: immediate hypersensitivity response Definition: An inflammatory response driven by antigen recognition by antibodies bound to Fc receptors on mast cells or basophils, occurring within minutes after exposure of a sensitized individual to the antigen, and leading to the release of a variety of inflammatory mediators such as histamines.